{
  "term_label": "Unknown biological process",
  "gene_name": "Endogenous retrovirus group K member 5 Gag polyprotein",
  "gene_symbol": "ERVK-5",
  "term_id": "UNKNOWN:0002",
  "gene": "UniProtKB:Q9HDB9"
}